{
  "term_id": "GO:0071763",
  "term_label": "nuclear membrane organization",
  "gene_symbol": "TOR1A",
  "gene_name": "Torsin-1A",
  "gene": "UniProtKB:O14656"
}